propionyl-CoA C2-trimethyltridecanoyltransferase activity [GO:0050632] (molecular function) Sources: RHEA:10408 Also known as: propionyl-CoA C(2)-trimethyltridecanoyltransferase activity, peroxisomal 3-oxoacyl coenzyme A thiolase, peroxisome sterol carrier protein thiolase, 3-oxopristanoyl-CoA hydrolase activity, 3-oxopristanoyl-CoA thiolase activity, 4,8,12-trimethyltridecanoyl-CoA:propanoyl-CoA 2-C-4,8,12-trimethyltridecanoyltransferase activity, 4,8,12-trimethyltridecanoyl-CoA:propanoyl-CoA C2-4,8,12-trimethyltridecanoyltransferase activity, SCPx, oxopristanoyl-CoA thiolase activity, sterol carrier protein, sterol carrier protein X-related thiolase activity Relationships: is a type of acyltransferase activity, transferring groups other than amino-acyl groups [GO:0016747] Definition: Catalysis of the reaction: 4,8,12-trimethyltridecanoyl-CoA + propanoyl-CoA = 3-oxopristanoyl-CoA + CoA.